L-arabinose 1-dehydrogenase (NAD+) activity [GO:0050022] (molecular function) Definition: Catalysis of the reaction: L-arabinose + NAD+ = L-arabinono-1,4-lactone + NADH. Also known as: L-arabinose 1-dehydrogenase activity, L-arabinose:NAD+ 1-oxidoreductase activity Relationships: is a type of GO:0016616 Sources: EC:1.1.1.46, MetaCyc:L-ARABINOSE-1-DEHYDROGENASE-RXN